inositol phosphate metabolic process [GO:0043647] (biological process) Definition: The chemical reactions and pathways involving inositol phosphate, 1,2,3,4,5,6-cyclohexanehexol, with one or more phosphate groups attached. Relationships: is a type of phosphate-containing compound metabolic process [GO:0006796]; is a type of organophosphate metabolic process [GO:0019637]; is a type of polyol metabolic process [GO:0019751] Subtypes: inositol trisphosphate metabolic process [GO:0032957], inositol phosphate biosynthetic process [GO:0032958], diphosphoinositol polyphosphate metabolic process [GO:0071543], inositol phosphate catabolic process [GO:0071545] Sources: GOC:jl Also known as: inositol phosphate metabolism, myo-inositol phosphate metabolic process, myo-inositol phosphate metabolism